{
  "gene_name": "Origin recognition complex subunit 4",
  "gene": "UniProtKB:O43929",
  "term_label": "DNA replication origin binding",
  "gene_symbol": "ORC4",
  "term_id": "GO:0003688"
}